{
  "gene": "UniProtKB:Q8NFZ5",
  "term_id": "GO:0034138",
  "gene_name": "TNFAIP3-interacting protein 2",
  "term_label": "toll-like receptor 3 signaling pathway",
  "gene_symbol": "TNIP2"
}